{
  "gene_name": "Defensin-6",
  "gene_symbol": "DEFA6",
  "term_label": "innate immune response",
  "term_id": "GO:0045087",
  "gene": "UniProtKB:Q01524"
}